dorsal fin morphogenesis [GO:0035142] (biological process) Definition: The process in which the anatomical structures of the dorsal fin are generated and organized. A dorsal fin is an unpaired medial fin on the dorsal aspect of fish that provides lateral stability while swimming. Generally fish have one or two dorsal fins. Sources: GOC:dgh Subtypes: embryonic dorsal fin morphogenesis [GO:0035123], GO:0035134 Relationships: is a type of GO:0035141; is part of dorsal fin development [GO:0033337]